{
  "gene_symbol": "PDZK1IP1",
  "gene_name": "PDZK1-interacting protein 1",
  "term_label": "Unknown molecular function",
  "term_id": "UNKNOWN:0001",
  "gene": "UniProtKB:Q13113"
}